lysosomal protein catabolic process [GO:1905146] (BP) Note: Also consider annotating to the term 'autophagy ; GO:0006914' or one of its descendants. References: PMID:24334770 Sources: GOC:PARL, GOC:TermGenie, GOC:bf, GO_REF:0000062 Definition: Any cellular protein catabolic process that takes place in a lysosome. Regulation: regulated by regulation of lysosomal protein catabolic process [GO:1905165]; negatively regulated by negative regulation of lysosomal protein catabolic process [GO:1905166]; positively regulated by positive regulation of lysosomal protein catabolic process [GO:1905167] Relationships: is a type of protein catabolic process in the vacuole [GO:0007039]; occurs in lysosome [GO:0005764] Also known as: cellular protein breakdown in lysosome, cellular protein catabolic process in lysosome, cellular protein catabolism in lysosome, cellular protein degradation in lysosome, lysosomal protein catabolism, lysosomal protein degradation, lysosomal proteolysis, proteolysis within lysosome